eukaryotic translation initiation factor 2alpha kinase activity [GO:0004694] (molecular function) Relationships: is a type of protein serine/threonine kinase activity [GO:0004674]; is part of regulation of translational initiation by eIF2 alpha phosphorylation [GO:0010998] Sources: GOC:mah, InterPro:IPR015516 Definition: Catalysis of the reaction: ATP + [eukaryotic translation initiation factor 2 alpha subunit] = ADP + [eukaryotic translation initiation factor 2 alpha subunit] phosphate.